{
  "gene_symbol": "SLCO2B1",
  "term_label": "basolateral plasma membrane",
  "gene": "UniProtKB:O94956",
  "term_id": "GO:0016323",
  "gene_name": "Solute carrier organic anion transporter family member 2B1"
}